{
  "gene": "UniProtKB:P46976",
  "term_id": "GO:0005737",
  "gene_symbol": "GYG1",
  "gene_name": "Glycogenin-1",
  "term_label": "cytoplasm"
}